{
  "gene_symbol": "CDC42EP1",
  "gene": "UniProtKB:Q00587",
  "gene_name": "Cdc42 effector protein 1",
  "term_id": "GO:0005856",
  "term_label": "cytoskeleton"
}